{
  "gene": "UniProtKB:Q6P435",
  "term_label": "Unknown molecular function",
  "gene_name": "Putative uncharacterized SMG1-like protein",
  "term_id": "UNKNOWN:0001",
  "gene_symbol": "Q6P435"
}